{
  "gene_name": "Sodium_glucose cotransporter 4",
  "gene_symbol": "SLC5A9",
  "term_id": "UNKNOWN:0002",
  "gene": "UniProtKB:Q2M3M2",
  "term_label": "Unknown biological process"
}